{
  "term_id": "GO:0005634",
  "term_label": "nucleus",
  "gene_name": "PRKC apoptosis WT1 regulator protein",
  "gene": "UniProtKB:Q96IZ0",
  "gene_symbol": "PAWR"
}